{
  "gene_symbol": "GGT7",
  "term_label": "plasma membrane",
  "gene_name": "Glutathione hydrolase 7",
  "term_id": "GO:0005886",
  "gene": "UniProtKB:Q9UJ14"
}